{
  "term_id": "UNKNOWN:0001",
  "gene_name": "Vitellogenin domain-containing protein",
  "gene": "UniProtKB:A0A8Q3SIG1",
  "gene_symbol": "LOC400499",
  "term_label": "Unknown molecular function"
}